{
  "gene_name": "Ankyrin repeat domain-containing protein 63",
  "term_label": "Unknown molecular function",
  "term_id": "UNKNOWN:0001",
  "gene": "UniProtKB:C9JTQ0",
  "gene_symbol": "ANKRD63"
}